{
  "gene": "UniProtKB:P59095",
  "gene_symbol": "STARD6",
  "term_id": "UNKNOWN:0001",
  "gene_name": "StAR-related lipid transfer protein 6",
  "term_label": "Unknown molecular function"
}